extrinsic component of postsynaptic recycling endosome membrane [GO:0099005] (cellular component) Relationships: is a type of extrinsic component of postsynaptic endosome membrane [GO:0098999]; is part of postsynaptic recycling endosome membrane [GO:0098944] Sources: GOC:autophagy, GOC:mf Definition: The component of the postsynaptic recycling endosome membrane consisting of gene products and protein complexes that are loosely bound to one of its surfaces, but not integrated into the hydrophobic region.